{
  "gene_name": "Cytochrome c oxidase assembly factor 6 homolog",
  "gene_symbol": "COA6",
  "term_label": "respiratory chain complex IV assembly",
  "gene": "UniProtKB:Q5JTJ3",
  "term_id": "GO:0008535"
}